{
  "term_label": "protein folding",
  "term_id": "GO:0006457",
  "gene_symbol": "DNAJB8",
  "gene": "UniProtKB:Q8NHS0",
  "gene_name": "DnaJ homolog subfamily B member 8"
}